{
  "term_id": "GO:0043066",
  "gene_name": "RAC-alpha serine_threonine-protein kinase",
  "term_label": "negative regulation of apoptotic process",
  "gene": "UniProtKB:P31749",
  "gene_symbol": "AKT1"
}